{
  "term_id": "GO:0008305",
  "gene_name": "Integrin alpha-3",
  "gene_symbol": "ITGA3",
  "term_label": "integrin complex",
  "gene": "UniProtKB:P26006"
}